regulation of lymphocyte mediated immunity [GO:0002706] (biological process) Subtypes: negative regulation of lymphocyte mediated immunity [GO:0002707], GO:0002708, regulation of T cell mediated immunity [GO:0002709], regulation of B cell mediated immunity [GO:0002712], GO:0002715 Definition: Any process that modulates the frequency, rate, or extent of lymphocyte mediated immunity. Relationships: is a type of regulation of leukocyte mediated immunity [GO:0002703]; regulates GO:0002449 Sources: GOC:add